NURF complex [GO:0016589] (cellular component) Also known as: nucleosome remodeling factor complex Relationships: is a type of ISWI-type complex [GO:0031010] Definition: An ISWI complex that contains an ATPase subunit of the ISWI family (SNF2L in mammals), a NURF301 homolog (BPTF in humans), and additional subunits, though the composition of these additional subunits varies slightly with species. NURF is involved in regulation of transcription from TRNA polymerase II promoters. References: PMID:10779516, PMID:11279013, PMID:15284901, PMID:16568949, PMID:21810179 Sources: GOC:bf, GOC:krc